establishment of endothelial barrier [GO:0061028] (biological process) Definition: The establishment of a barrier between endothelial cell layers, such as those in the brain, lung or intestine, to exert specific and selective control over the passage of water and solutes, thus allowing formation and maintenance of compartments that differ in fluid and solute composition. Subtypes: establishment of endothelial blood-brain barrier [GO:0014045], establishment of endothelial intestinal barrier [GO:0090557] Relationships: is a type of endothelial cell development [GO:0001885] Regulation: regulated by GO:1903140; negatively regulated by negative regulation of establishment of endothelial barrier [GO:1903141]; positively regulated by positive regulation of establishment of endothelial barrier [GO:1903142] Sources: GOC:dph